asparagine metabolic process [GO:0006528] (biological process) Also known as: asparagine metabolism Definition: The chemical reactions and pathways involving asparagine, 2-amino-3-carbamoylpropanoic acid. Relationships: is a type of GO:0019752 Sources: GOC:go_curators Subtypes: cyclization of asparagine involved in intein-mediated protein splicing [GO:0019801], L-asparagine metabolic process [GO:0070982]